amyloplast membrane [GO:0033097] (cellular component) Definition: Either of the lipid bilayers that surround an amyloplast and form the amyloplast envelope. Sources: GOC:ecd Relationships: is a type of plastid membrane [GO:0042170]; is part of amyloplast envelope [GO:0033096] Subtypes: amyloplast inner membrane [GO:0033098]